telencephalon regionalization [GO:0021978] (biological process) Relationships: is a type of regionalization [GO:0003002]; is part of telencephalon development [GO:0021537]; is part of forebrain regionalization [GO:0021871] Definition: The regionalization process that creates areas within the forebrain that will direct the behavior of cell migration in differentiation as the telencephalon develops. Sources: GOC:cls, GOC:dgh, GOC:dph, GOC:jid, GOC:mgi_curators